negative regulation of uterine smooth muscle contraction [GO:0070473] (biological process) Definition: Any process that decreases the frequency, rate or extent of uterine smooth muscle contraction. Sources: GOC:go_curators Also known as: down regulation of uterine smooth muscle contraction, down-regulation of uterine smooth muscle contraction, downregulation of uterine smooth muscle contraction, negative regulation of myometrial contraction, negative regulation of myometrial smooth muscle contraction, negative regulation of myometrium contraction, inhibition of uterine smooth muscle contraction, uterine smooth muscle relaxation Relationships: is a type of negative regulation of smooth muscle contraction [GO:0045986]; is a type of regulation of uterine smooth muscle contraction [GO:0070472]; RO_0002212 uterine smooth muscle contraction [GO:0070471]